{
  "gene": "UniProtKB:Q02246",
  "term_label": "cell-cell adhesion mediator activity",
  "gene_name": "Contactin-2",
  "gene_symbol": "CNTN2",
  "term_id": "GO:0098632"
}